{
  "term_label": "actin filament binding",
  "gene": "UniProtKB:P35580",
  "gene_symbol": "MYH10",
  "term_id": "GO:0051015",
  "gene_name": "Myosin-10"
}